{
  "gene_name": "Kinesin-like protein KIF7",
  "term_id": "GO:0005871",
  "term_label": "kinesin complex",
  "gene": "UniProtKB:Q2M1P5",
  "gene_symbol": "KIF7"
}